{
  "term_label": "thiamine transport",
  "gene_symbol": "SLC19A2",
  "gene_name": "Thiamine transporter 1",
  "gene": "UniProtKB:O60779",
  "term_id": "GO:0015888"
}